{
  "term_id": "UNKNOWN:0001",
  "gene": "UniProtKB:Q6YI46",
  "term_label": "Unknown molecular function",
  "gene_name": "Transmembrane protein 64",
  "gene_symbol": "TMEM64"
}